{
  "gene": "UniProtKB:Q9Y258",
  "gene_name": "C-C motif chemokine 26",
  "term_id": "GO:0048245",
  "gene_symbol": "CCL26",
  "term_label": "eosinophil chemotaxis"
}